{
  "gene": "UniProtKB:Q9BQA1",
  "term_label": "Unknown biological process",
  "gene_symbol": "WDR77",
  "gene_name": "Methylosome protein WDR77",
  "term_id": "UNKNOWN:0002"
}